{
  "term_label": "intracellular protein localization",
  "gene_name": "Septin-14",
  "gene_symbol": "SEPTIN14",
  "term_id": "GO:0008104",
  "gene": "UniProtKB:Q6ZU15"
}